{
  "gene": "UniProtKB:Q9Y5W5",
  "term_label": "cell surface",
  "gene_name": "Wnt inhibitory factor 1",
  "gene_symbol": "WIF1",
  "term_id": "GO:0009986"
}